positive thymic T cell selection [GO:0045059] (biological process) Definition: The process of sparing immature T cells in the thymus which react with self-MHC protein complexes with low affinity levels from apoptotic death. Regulation: regulated by regulation of positive thymic T cell selection [GO:1902232]; negatively regulated by negative regulation of positive thymic T cell selection [GO:1902233]; positively regulated by positive regulation of positive thymic T cell selection [GO:1902234] Relationships: is a type of positive T cell selection [GO:0043368]; is a type of thymic T cell selection [GO:0045061] References: PMID:12414722 Sources: ISBN:0781735149 Also known as: positive thymic T lymphocyte selection, positive thymic T-cell selection, positive thymic T-lymphocyte selection